{
  "term_label": "oocyte development",
  "gene_name": "GATA-type zinc finger protein 1",
  "gene_symbol": "ZGLP1",
  "gene": "UniProtKB:P0C6A0",
  "term_id": "GO:0048599"
}